cellular response to acetylcholine [GO:1905145] (biological process) References: PMID:21238497 Sources: GOC:TermGenie, GO_REF:0000071 Relationships: is a type of cellular response to nitrogen compound [GO:1901699]; is a type of cellular response to oxygen-containing compound [GO:1901701]; is a type of GO:1905144 Definition: Any process that results in a change in state or activity of a cell (in terms of movement, secretion, enzyme production, gene expression, etc.) as a result of an acetylcholine stimulus.